{
  "term_id": "GO:0004938",
  "gene": "UniProtKB:P18825",
  "gene_symbol": "ADRA2C",
  "gene_name": "Alpha-2C adrenergic receptor",
  "term_label": "alpha2-adrenergic receptor activity"
}